5'-3' RNA polymerase activity [GO:0034062] (molecular function) Also known as: RNA polymerase activity Relationships: is a type of RNA polymerase activity [GO:0097747] Definition: Catalysis of the reaction: nucleoside triphosphate + RNA(n) = diphosphate + RNA(n+1); the synthesis of RNA from ribonucleotide triphosphates in the presence of a nucleic acid template, via extension of the 3'-end. Sources: GOC:mah, GOC:pf, RHEA:21248 Subtypes: DNA-directed RNA polymerase activity [GO:0003899], RNA-directed RNA polymerase activity [GO:0003968]